reservosome membrane [GO:0106126] (cellular component) Relationships: is a type of cellular anatomical structure [GO:0110165]; is part of reservosome [GO:0106123] Definition: The lipid bilayer surrounding a reservosome. References: PMID:12204365, PMID:15521631, PMID:18452191, PMID:19288526, PMID:21818313, PMID:22425988 Sources: GOC:ach